positive regulation of behavior [GO:0048520] (biological process) Definition: Any process that activates or increases the frequency, rate or extent of behavior, the internally coordinated responses (actions or inactions) of whole living organisms (individuals or groups) to internal or external stimuli. Relationships: is a type of GO:0050795; is a type of positive regulation of multicellular organismal process [GO:0051240]; RO_0002213 behavior [GO:0007610] Sources: GOC:jid, GOC:pr Subtypes: positive regulation of circadian sleep/wake cycle, wakefulness [GO:0010841], positive regulation of host-seeking behavior [GO:0032540], positive regulation of circadian sleep/wake cycle, sleep [GO:0045938], positive regulation of locomotion involved in locomotory behavior [GO:0090326], positive regulation of egg-laying behavior [GO:1901046], positive regulation of male mating behavior [GO:1902437], positive regulation of foraging behavior [GO:1903370], positive regulation of locomotor rhythm [GO:1904061], positive regulation of mechanosensory behavior [GO:1905792], positive regulation of feeding behavior [GO:2000253], positive regulation of behavioral fear response [GO:2000987] Also known as: up regulation of behavior, up-regulation of behavior, upregulation of behavior, activation of behavior, stimulation of behavior